{
  "gene": "UniProtKB:Q8TCX1",
  "gene_name": "Cytoplasmic dynein 2 light intermediate chain 1",
  "gene_symbol": "DYNC2LI1",
  "term_id": "GO:0005930",
  "term_label": "axoneme"
}